{
  "gene_symbol": "MEDAG",
  "term_label": "cytoplasm",
  "gene_name": "Mesenteric estrogen-dependent adipogenesis protein",
  "gene": "UniProtKB:Q5VYS4",
  "term_id": "GO:0005737"
}